{
  "gene_symbol": "CFB",
  "gene_name": "Complement factor B",
  "term_label": "complement activation, alternative pathway",
  "gene": "UniProtKB:P00751",
  "term_id": "GO:0006957"
}